{
  "gene": "UniProtKB:Q16760",
  "gene_symbol": "DGKD",
  "term_label": "diacylglycerol metabolic process",
  "gene_name": "Diacylglycerol kinase delta",
  "term_id": "GO:0046339"
}